regulation of vesicle targeting, to, from or within Golgi [GO:0048209] (biological process) Relationships: is a type of regulation of cellular localization [GO:0060341]; regulates vesicle targeting, to, from or within Golgi [GO:0048199] Also known as: regulation of Golgi vesicle targeting Definition: Any process that modulates the frequency, rate, or destination of vesicle-mediated transport to, from or within the Golgi apparatus. References: PMID:10219233 Sources: GOC:jid, GOC:mah, ISBN:0716731363